regulation of transcription of nucleolar large rRNA by RNA polymerase I [GO:1901836] (biological process) Sources: GOC:TermGenie, GOC:sart Definition: Any process that modulates the frequency, rate or extent of transcription of nuclear large rRNA mediated by RNA polymerase I. Relationships: is a type of GO:0006356; regulates GO:0042790 Also known as: regulation of transcription of nuclear large rRNA transcript from RNA polymerase I promoter, regulation of transcription of nuclear rRNA large Pol I transcript Subtypes: negative regulation of transcription of nucleolar large rRNA by RNA polymerase I [GO:1901837], positive regulation of transcription of nucleolar large rRNA by RNA polymerase I [GO:1901838]